{
  "gene_symbol": "FOXL2",
  "gene_name": "Forkhead box protein L2",
  "gene": "UniProtKB:P58012",
  "term_id": "UNKNOWN:0003",
  "term_label": "Unknown cellular component"
}